gastric emptying [GO:0035483] (biological process) Sources: GOC:cy, ISBN:9781416032458 Definition: The process in which the liquid and liquid-suspended solid contents of the stomach exit through the pylorus into the duodenum. Relationships: is a type of gastric motility [GO:0035482] Regulation: regulated by regulation of gastric emptying [GO:0120060]; negatively regulated by GO:0120061; positively regulated by positive regulation of gastric emptying [GO:0120062]